{
  "gene_name": "Myotubularin-related protein 11",
  "term_label": "membrane",
  "term_id": "GO:0016020",
  "gene_symbol": "MTMR11",
  "gene": "UniProtKB:A4FU01"
}